{
  "gene": "UniProtKB:P48163",
  "gene_name": "NADP-dependent malic enzyme",
  "term_id": "GO:0005739",
  "term_label": "mitochondrion",
  "gene_symbol": "ME1"
}